{
  "gene_symbol": "NME3",
  "gene_name": "Nucleoside diphosphate kinase 3",
  "term_id": "UNKNOWN:0002",
  "term_label": "Unknown biological process",
  "gene": "UniProtKB:Q13232"
}